{
  "term_label": "DNA-binding transcription factor activity, RNA polymerase II-specific",
  "term_id": "GO:0000981",
  "gene_name": "Zinc finger protein 577",
  "gene": "UniProtKB:Q9BSK1",
  "gene_symbol": "ZNF577"
}